NACHT domain binding [GO:0032089] (molecular function) Relationships: is a type of GO:0019904 Sources: GOC:rl Definition: Binding to a NACHT (NAIP, CIITA, HET-E and TP1) domain. The NACHT domain consists of seven distinct conserved motifs, including an ATP/GTPase specific P-loop, a Mg2+-binding site and five more specific motifs.